{
  "gene_symbol": "ZNF471",
  "gene": "UniProtKB:Q9BX82",
  "term_label": "DNA-binding transcription factor activity, RNA polymerase II-specific",
  "term_id": "GO:0000981",
  "gene_name": "Zinc finger protein 471"
}